dehydroascorbic acid transmembrane transporter activity [GO:0033300] (molecular function) Relationships: is_a vitamin transmembrane transporter activity [GO:0090482]; is part of dehydroascorbic acid transport [GO:0070837] Sources: GOC:go_curators Definition: Enables the transfer of dehydroascorbate, 5-(1,2-dihydroxyethyl)furan-2,3,4(5H)-trione, from one side of a membrane to the other. Also known as: dehydroascorbate transporter activity, dehydroascorbic acid transporter activity